{
  "gene_name": "Troponin I, fast skeletal muscle",
  "gene": "UniProtKB:P48788",
  "term_label": "skeletal muscle contraction",
  "gene_symbol": "TNNI2",
  "term_id": "GO:0003009"
}